{
  "gene": "UniProtKB:P05556",
  "gene_symbol": "ITGB1",
  "gene_name": "Integrin beta-1",
  "term_id": "GO:0008305",
  "term_label": "integrin complex"
}